{
  "term_label": "Unknown cellular component",
  "gene_name": "Putative protein FAM86JP",
  "gene_symbol": "FAM86JP",
  "term_id": "UNKNOWN:0003",
  "gene": "UniProtKB:Q05BU3"
}